{
  "term_label": "cytoplasm",
  "gene": "UniProtKB:P51677",
  "term_id": "GO:0005737",
  "gene_symbol": "CCR3",
  "gene_name": "C-C chemokine receptor type 3"
}